{
  "term_label": "5S class rRNA transcription by RNA polymerase III",
  "gene": "UniProtKB:Q12789",
  "term_id": "GO:0042791",
  "gene_name": "General transcription factor 3C polypeptide 1",
  "gene_symbol": "GTF3C1"
}